dATP biosynthetic process [GO:0006175] (biological process) Definition: The chemical reactions and pathways resulting in the formation of dATP, deoxyadenosine triphosphate (2'-deoxyadenosine 5'-triphosphate). Sources: ISBN:0198506732 Subtypes: GO:0006176 Relationships: is a type of purine deoxyribonucleotide biosynthetic process [GO:0009153]; is a type of purine deoxyribonucleoside triphosphate biosynthetic process [GO:0009216]; is a type of dATP metabolic process [GO:0046060] Also known as: dATP anabolism, dATP biosynthesis, dATP formation, dATP synthesis